{
  "term_label": "ciliary rootlet",
  "gene_symbol": "ODAD3",
  "gene": "UniProtKB:A5D8V7",
  "term_id": "GO:0035253",
  "gene_name": "Outer dynein arm-docking complex subunit 3"
}